protein-phycourobilin linkage [GO:0017010] (biological process) Definition: The linkage of the chromophore phycourobilin to phycoerythrins. Relationships: is a type of protein-bilin linkage [GO:0017007] Sources: RESID:AA0260